{
  "term_label": "Unknown biological process",
  "term_id": "UNKNOWN:0002",
  "gene": "UniProtKB:Q5T8R8",
  "gene_symbol": "DOCK8-AS1",
  "gene_name": "Uncharacterized protein DOCK8-AS1"
}